rectal diverticulum development [GO:0039009] (biological process) Definition: The process whose specific outcome is the progression of the rectal diverticulum over time, from its formation to the mature structure. The rectal diverticulum is an outgrowth of the cloaca and links the pronephric kidney to the exterior. Also known as: pronephric rectal diverticulum development Relationships: is a type of GO:0048856; is part of pronephros development [GO:0048793] References: PMID:10535314, PMID:18226983 Sources: GOC:mtg_kidney_jan10, XAO:0001015